T cell selection [GO:0045058] (biological process) Subtypes: beta selection [GO:0043366], GO:0043368, negative T cell selection [GO:0043383], GO:0045061, GO:0045062 Also known as: T lymphocyte selection, T-cell selection, T-lymphocyte selection References: PMID:12414722 Sources: ISBN:0781735149 Definition: The process in which T cells that express T cell receptors that are restricted by self MHC protein complexes and tolerant to self antigens are selected for further maturation. Relationships: is a type of immune system process [GO:0002376]; is part of T cell differentiation [GO:0030217]